{
  "gene_name": "Tropomodulin-3",
  "term_id": "GO:0005865",
  "term_label": "striated muscle thin filament",
  "gene": "UniProtKB:Q9NYL9",
  "gene_symbol": "TMOD3"
}